{
  "term_id": "GO:0005615",
  "gene_symbol": "FCN1",
  "term_label": "extracellular space",
  "gene": "UniProtKB:O00602",
  "gene_name": "Ficolin-1"
}